mitotic spindle assembly checkpoint signaling [GO:0007094] (biological process) References: PMID:12360190 Sources: GOC:mtg_cell_cycle Also known as: mitotic cell cycle spindle assembly checkpoint, mitotic checkpoint, mitotic spindle assembly checkpoint, mitotic spindle assembly checkpoint signalling, signal transduction involved in mitotic cell cycle spindle assembly checkpoint, signal transduction involved in mitotic spindle assembly checkpoint, Dma1-dependent checkpoint, Mad2-dependent checkpoint, SAC-independent checkpoint, signal transduction involved in Dma1-dependent checkpoint, signal transduction involved in SAC-independent checkpoint, signaling cascade involved in Dma1-dependent checkpoint, signaling cascade involved in SAC-independent checkpoint, signalling cascade involved in Dma1-dependent checkpoint, signalling cascade involved in SAC-independent checkpoint, signaling pathway involved in Dma1-dependent checkpoint, signaling pathway involved in SAC-independent checkpoint, signalling pathway involved in Dma1-dependent checkpoint, signalling pathway involved in SAC-independent checkpoint Regulation: regulated by regulation of mitotic cell cycle spindle assembly checkpoint [GO:0090266]; positively regulated by positive regulation of mitotic cell cycle spindle assembly checkpoint [GO:0090267]; negatively regulated by negative regulation of mitotic spindle assembly checkpoint signaling [GO:0140499] Definition: A mitotic cell cycle checkpoint that delays mitotic sister chromatid separation and consequently the mitotic metaphase/anaphase transition until the spindle is correctly assembled and chromosomes are attached to the spindle. Spindle assembly checkpoint signaling begins with the activated Mph family kinase, and results in the inhibition of the Anaphase Promoting Complex and its activator Sleepy/Cdc20 by the mitotic checkpoint complex (MCC). Relationships: is a type of GO:0045841; is a type of spindle assembly checkpoint signaling [GO:0071173]; is a type of mitotic spindle checkpoint signaling [GO:0071174]